testosterone secretion [GO:0035936] (biological process) Regulation: regulated by regulation of testosterone secretion [GO:2000843]; negatively regulated by GO:2000844; positively regulated by positive regulation of testosterone secretion [GO:2000845] Definition: The regulated release of testosterone into the circulatory system. Testosterone is an androgen having 17beta-hydroxy and 3-oxo groups, together with unsaturation at C-4-C-5. References: PMID:12606499 Sources: GOC:sl Relationships: is a type of organic hydroxy compound transport [GO:0015850]; is a type of hormone secretion [GO:0046879]; is a type of lipid export from cell [GO:0140353]